UFM1 activating enzyme activity [GO:0071566] (molecular function) References: PMID:20018847 Sources: GOC:sp Definition: Catalysis of the activation of the small ubiquitin-related modifier UFM1, through the formation of an ATP-dependent high-energy thiolester bond. Relationships: is a type of ubiquitin-like modifier activating enzyme activity [GO:0008641]